{
  "gene_symbol": "NXN",
  "gene": "UniProtKB:Q6DKJ4",
  "term_label": "thioredoxin-disulfide reductase (NADPH) activity",
  "term_id": "GO:0004791",
  "gene_name": "Nucleoredoxin"
}